{
  "term_id": "GO:0051123",
  "term_label": "RNA polymerase II preinitiation complex assembly",
  "gene_symbol": "TAF12",
  "gene_name": "Transcription initiation factor TFIID subunit 12",
  "gene": "UniProtKB:Q16514"
}